{
  "term_label": "Unknown cellular component",
  "gene": "UniProtKB:A0A0A0MT96",
  "term_id": "UNKNOWN:0003",
  "gene_symbol": "IGKJ3",
  "gene_name": "Immunoglobulin kappa joining 3 (Fragment)"
}